{
  "term_id": "GO:0055008",
  "gene": "UniProtKB:O15273",
  "gene_name": "Telethonin",
  "gene_symbol": "TCAP",
  "term_label": "cardiac muscle tissue morphogenesis"
}